{
  "gene_symbol": "PACS1",
  "term_id": "GO:0044325",
  "term_label": "transmembrane transporter binding",
  "gene_name": "Phosphofurin acidic cluster sorting protein 1",
  "gene": "UniProtKB:Q6VY07"
}